{
  "term_id": "GO:0003779",
  "term_label": "actin binding",
  "gene": "UniProtKB:Q8TE67",
  "gene_name": "Epidermal growth factor receptor kinase substrate 8-like protein 3",
  "gene_symbol": "EPS8L3"
}